{
  "gene": "UniProtKB:Q6NYC1",
  "term_label": "nucleus",
  "gene_symbol": "JMJD6",
  "gene_name": "Bifunctional arginine demethylase and lysyl-hydroxylase JMJD6",
  "term_id": "GO:0005634"
}